{
  "gene_name": "Interferon-induced protein with tetratricopeptide repeats 5",
  "gene": "UniProtKB:Q13325",
  "term_id": "GO:0071345",
  "gene_symbol": "IFIT5",
  "term_label": "cellular response to cytokine stimulus"
}